{
  "gene_name": "Gamma-tubulin complex component 4",
  "term_label": "meiotic cell cycle",
  "term_id": "GO:0051321",
  "gene_symbol": "TUBGCP4",
  "gene": "UniProtKB:Q9UGJ1"
}